regulation of arabinoxylan-containing compound catabolic process [GO:2000921] (BP) Relationships: is a type of regulation of xylan catabolic process [GO:2001000]; regulates GO:2000888 Definition: Any process that modulates the frequency, rate or extent of arabinoxylan-containing compound catabolic process. Subtypes: regulation of glucuronoarabinoxylan catabolic process [GO:2000918], negative regulation of arabinoxylan-containing compound catabolic process [GO:2000922], GO:2000923 Also known as: regulation of arabinoxylan catabolism Sources: GOC:mengo_curators